galactoxylomannan biosynthetic process [GO:0062191] (biological process) Also known as: GalXM biosynthetic process, galactoxylomannan anabolism, galactoxylomannan biosynthesis, galactoxylomannan formation, galactoxylomannan synthesis, glucuronoxylomannogalactan biosynthetic process Relationships: is a type of fungal-type cell wall polysaccharide biosynthetic process [GO:0051278] Definition: The chemical reactions and pathways resulting in the formation of the exopolysaccharide galactoxylomannan. Galactoxylomannan is produced by a pathogenic fungus and causes paralysis in some animals. References: PMID:16441437, PMID:18952901, PMID:19684080, PMID:21843086